{
  "gene": "UniProtKB:P25685",
  "term_label": "Hsp70 protein binding",
  "gene_symbol": "DNAJB1",
  "gene_name": "DnaJ homolog subfamily B member 1",
  "term_id": "GO:0030544"
}